{
  "term_id": "GO:0016887",
  "gene_name": "Vacuolar protein sorting-associated protein 4A",
  "gene": "UniProtKB:Q9UN37",
  "term_label": "ATP hydrolysis activity",
  "gene_symbol": "VPS4A"
}